{
  "term_label": "cyclin-dependent protein serine/threonine kinase regulator activity",
  "term_id": "GO:0016538",
  "gene_name": "Protein CNPPD1",
  "gene_symbol": "CNPPD1",
  "gene": "UniProtKB:Q9BV87"
}